{
  "gene_symbol": "OR2G2",
  "term_id": "GO:0005886",
  "gene_name": "Olfactory receptor 2G2",
  "term_label": "plasma membrane",
  "gene": "UniProtKB:Q8NGZ5"
}